effector-mediated suppression of host salicylic acid-mediated innate immune signaling [GO:0140502] (biological process) Relationships: is a type of symbiont-mediated suppression of defense-related host salicylic acid-mediated signal transduction pathway [GO:0052003]; is a type of GO:0052029; is a type of effector-mediated perturbation of host innate immune response by symbiont [GO:0140404] References: PMID:25438793, PMID:30651637 Also known as: effector-mediated disruption of host salicylic acid-mediated innate immune signalling, effector-mediated suppression of host salicylic acid-mediated innate immune signalling Definition: A process mediated by a molecule secreted by a symbiont that results in the suppression of host salicylic acid-mediated innate immune signaling.